{
  "gene": "UniProtKB:P42574",
  "term_label": "cysteine-type endopeptidase activity",
  "term_id": "GO:0004197",
  "gene_name": "Caspase-3",
  "gene_symbol": "CASP3"
}